{
  "gene_name": "Arylsulfatase F",
  "gene": "UniProtKB:P54793",
  "term_label": "Unknown cellular component",
  "gene_symbol": "ARSF",
  "term_id": "UNKNOWN:0003"
}